type 2A serotonin receptor binding [GO:0031826] (molecular function) Definition: Binding to a type 2A serotonin receptor. Sources: GOC:mah, GOC:nln Also known as: 5-hydroxytryptamine 2A receptor binding, type 2A serotonin receptor ligand Relationships: is a type of G protein-coupled serotonin receptor binding [GO:0031821]